{
  "term_id": "GO:0005200",
  "gene_name": "Tubulin alpha chain-like 3",
  "term_label": "structural constituent of cytoskeleton",
  "gene": "UniProtKB:A6NHL2",
  "gene_symbol": "TUBAL3"
}